trimethylamine-N-oxide reductase (cytochrome c) activity [GO:0050626] (molecular function) Also known as: TMAO reductase activity, TOR activity, trimethylamine:cytochrome c oxidoreductase activity Sources: EC:1.7.2.3, MetaCyc:1.7.2.3-RXN Relationships: is a type of oxidoreductase activity, acting on other nitrogenous compounds as donors, cytochrome as acceptor [GO:0016662] Definition: Catalysis of the reaction: trimethylamine + 2 (ferricytochrome c)-subunit + H2O = trimethylamine-N-oxide + 2 (ferrocytochrome c)-subunit + 2 H+.